{
  "gene": "UniProtKB:Q9BV94",
  "gene_name": "ER degradation-enhancing alpha-mannosidase-like protein 2",
  "gene_symbol": "EDEM2",
  "term_label": "ubiquitin-dependent glycoprotein ERAD pathway",
  "term_id": "GO:0097466"
}